{
  "term_label": "DNA-binding transcription factor activity",
  "gene": "UniProtKB:A6NNF4",
  "gene_name": "Zinc finger protein 726",
  "gene_symbol": "ZNF726",
  "term_id": "GO:0003700"
}